terpene synthase activity [GO:0010333] (molecular function) Definition: Catalysis of the formation of cyclic terpenes through the cyclization of linear terpenes (e.g. isopentenyl-PP, geranyl-PP, farnesyl-PP and geranylgeranyl-PP) containing varying numbers of isoprene units. Sources: GOC:tair_curators Relationships: is a type of carbon-oxygen lyase activity, acting on phosphates [GO:0016838] Subtypes: ent-kaurene synthase activity [GO:0009899], sesquiterpene synthase activity [GO:0010334], GO:0034002, GO:0034009, ent-isokaurene synthase activity [GO:0034281], casbene synthase activity [GO:0050449], pinene synthase activity [GO:0050550], myrcene synthase activity [GO:0050551], GO:0050552, sabinene synthase activity [GO:0080015], GO:0106100